{
  "gene_symbol": "CPZ",
  "gene": "UniProtKB:Q66K79",
  "term_label": "extracellular space",
  "term_id": "GO:0005615",
  "gene_name": "Carboxypeptidase Z"
}